{
  "term_label": "dendrite membrane",
  "term_id": "GO:0032590",
  "gene": "UniProtKB:Q14003",
  "gene_name": "Potassium voltage-gated channel subfamily C member 3",
  "gene_symbol": "KCNC3"
}